{
  "term_label": "Unknown molecular function",
  "gene": "UniProtKB:Q9BPY8",
  "gene_name": "Homeodomain-only protein",
  "gene_symbol": "HOPX",
  "term_id": "UNKNOWN:0001"
}